{
  "term_label": "interleukin-11 receptor activity",
  "gene_name": "Ciliary neurotrophic factor receptor subunit alpha",
  "gene": "UniProtKB:P26992",
  "term_id": "GO:0004921",
  "gene_symbol": "CNTFR"
}